centromere clustering at the mitotic interphase nuclear envelope [GO:0072766] (biological process) Also known as: centromere clustering at the nuclear periphery, centromere-SPB clustering, kinetochore clustering at SPB, kinetochore clustering at spindle pole body, kinetochore localization at spindle pole body, kinetochore clustering at the old mitotic spindle pole body, centromere clustering at the mitotic nuclear envelope, rabl configuration References: PMID:21965289, PMID:23166349 Sources: GOC:mah, GOC:vw Definition: The process in which chromatin, or kinetochores are anchored to the nuclear envelope. This process involves the microtubule cytoskeleton, and nuclear tethering factors and is responsible for the Rabl-like configuration of chromosomes in the interphase nuclei. Relationships: is a type of chromosome attachment to the nuclear envelope [GO:0097240]; is a type of centromere clustering [GO:0098653]; is a type of GO:1903047